{
  "gene_symbol": "GGTLC1",
  "gene": "UniProtKB:Q9BX51",
  "gene_name": "Glutathione hydrolase light chain 1",
  "term_label": "Unknown biological process",
  "term_id": "UNKNOWN:0002"
}